{
  "gene": "UniProtKB:Q5VZ46",
  "gene_symbol": "KIAA1614",
  "term_id": "GO:0005634",
  "term_label": "nucleus",
  "gene_name": "Uncharacterized protein KIAA1614"
}